{
  "term_id": "GO:0030425",
  "gene_symbol": "PENK",
  "gene": "UniProtKB:P01210",
  "gene_name": "Proenkephalin-A",
  "term_label": "dendrite"
}